gamma-glutamyl-peptidase activity [GO:0034722] (molecular function) Also known as: gamma-glutamyl hydrolase activity Relationships: is_a cysteine-type peptidase activity [GO:0008234]; is a type of omega peptidase activity [GO:0008242] Sources: EC:3.4.19.9, MEROPS_fam:C26 Definition: Catalysis of the cleavage of a gamma-linked glutamate bond.